positive regulation of alcohol biosynthetic process [GO:1902932] (biological process) Definition: Any process that activates or increases the frequency, rate or extent of alcohol biosynthetic process. References: PMID:23332010 Sources: GOC:TermGenie, GOC:mengo_curators, GO_REF:0000058 Relationships: is a type of GO:0009891; is a type of positive regulation of small molecule metabolic process [GO:0062013]; is a type of regulation of alcohol biosynthetic process [GO:1902930]; positively regulates alcohol biosynthetic process [GO:0046165] Subtypes: positive regulation of abscisic acid biosynthetic process [GO:0010116], positive regulation of aldosterone biosynthetic process [GO:0032349], positive regulation of cholesterol biosynthetic process [GO:0045542], positive regulation of inositol phosphate biosynthetic process [GO:0060732], GO:0070452, positive regulation of thiamine biosynthetic process [GO:0090180], GO:0140724, positive regulation terrein biosynthetic process [GO:0140881], positive regulation of inositol biosynthetic process [GO:1900090], positive regulation of kojic acid biosynthetic process [GO:1900396], positive regulation of butyryl-CoA catabolic process to butanol [GO:1900499], positive regulation of asperfuranone biosynthetic process [GO:1900639], positive regulation of neosartoricin biosynthetic process [GO:1902055], positive regulation of phytol biosynthetic process [GO:1904964], positive regulation of cortisol biosynthetic process [GO:2000066] Also known as: positive regulation of solventogenesis, positive regulation of alcohol anabolism, positive regulation of alcohol biosynthesis, positive regulation of alcohol formation, positive regulation of alcohol synthesis, up regulation of alcohol anabolism, up regulation of alcohol biosynthesis, up regulation of alcohol biosynthetic process, up regulation of alcohol formation, up regulation of alcohol synthesis, up-regulation of alcohol anabolism, up-regulation of alcohol biosynthesis, up-regulation of alcohol biosynthetic process, up-regulation of alcohol formation, up-regulation of alcohol synthesis, upregulation of alcohol anabolism, upregulation of alcohol biosynthesis, upregulation of alcohol biosynthetic process, upregulation of alcohol formation, upregulation of alcohol synthesis, activation of alcohol anabolism, activation of alcohol biosynthesis, activation of alcohol biosynthetic process, activation of alcohol formation, activation of alcohol synthesis